{
  "gene_name": "ORM1-like protein 1",
  "term_label": "ceramide metabolic process",
  "term_id": "GO:0006672",
  "gene_symbol": "ORMDL1",
  "gene": "UniProtKB:Q9P0S3"
}